{
  "gene_name": "Possible J 10 gene (Fragment)",
  "gene_symbol": "TRAJ10",
  "gene": "UniProtKB:A0N4Z7",
  "term_id": "UNKNOWN:0001",
  "term_label": "Unknown molecular function"
}